{
  "term_label": "phosphatidylinositol phosphate binding",
  "gene": "UniProtKB:Q6P3S1",
  "term_id": "GO:1901981",
  "gene_symbol": "DENND1B",
  "gene_name": "DENN domain-containing protein 1B"
}